{
  "term_id": "GO:0031012",
  "gene": "UniProtKB:Q8N8U9",
  "gene_symbol": "BMPER",
  "gene_name": "BMP-binding endothelial regulator protein",
  "term_label": "extracellular matrix"
}